positive regulation of phosphodiesterase I activity [GO:1902800] (biological process) References: PMID:24559510 Sources: GOC:TermGenie, GO_REF:0000059 Definition: Any process that activates or increases the frequency, rate or extent of phosphodiesterase I activity. Also known as: positive regulation of 5' nucleotide phosphodiesterase/alkaline phosphodiesterase I activity, positive regulation of PDE I activity, positive regulation of nucleotide pyrophosphatase/phosphodiesterase I activity, positive regulation of oligonucleate 5'-nucleotidohydrolase activity, positive regulation of orthophosphoric diester phosphohydrolase activity, up regulation of 5' nucleotide phosphodiesterase/alkaline phosphodiesterase I activity, up regulation of PDE I activity, up regulation of nucleotide pyrophosphatase/phosphodiesterase I activity, up regulation of oligonucleate 5'-nucleotidohydrolase activity, up regulation of orthophosphoric diester phosphohydrolase activity, up regulation of phosphodiesterase I activity, up-regulation of 5' nucleotide phosphodiesterase/alkaline phosphodiesterase I activity, up-regulation of PDE I activity, up-regulation of nucleotide pyrophosphatase/phosphodiesterase I activity, up-regulation of oligonucleate 5'-nucleotidohydrolase activity, up-regulation of orthophosphoric diester phosphohydrolase activity, up-regulation of phosphodiesterase I activity, upregulation of 5' nucleotide phosphodiesterase/alkaline phosphodiesterase I activity, upregulation of PDE I activity, upregulation of nucleotide pyrophosphatase/phosphodiesterase I activity, upregulation of oligonucleate 5'-nucleotidohydrolase activity, upregulation of orthophosphoric diester phosphohydrolase activity, upregulation of phosphodiesterase I activity, activation of 5' nucleotide phosphodiesterase/alkaline phosphodiesterase I activity, activation of PDE I activity, activation of nucleotide pyrophosphatase/phosphodiesterase I activity, activation of oligonucleate 5'-nucleotidohydrolase activity, activation of orthophosphoric diester phosphohydrolase activity, activation of phosphodiesterase I activity, activation of 5'-NPDase activity, activation of 5'-PDE activity, activation of 5'-PDase activity, activation of 5'-exonuclease activity, activation of 5'-nucleotide phosphodiesterase activity, activation of 5'-phosphodiesterase activity, activation of 5'NPDE activity, activation of alkaline phosphodiesterase activity, activation of exonuclease I activity, positive regulation of 5'-NPDase activity, positive regulation of 5'-PDE activity, positive regulation of 5'-PDase activity, positive regulation of 5'-exonuclease activity, positive regulation of 5'-nucleotide phosphodiesterase activity, positive regulation of 5'-phosphodiesterase activity, positive regulation of 5'NPDE activity, positive regulation of alkaline phosphodiesterase activity, positive regulation of exonuclease I activity, up regulation of 5'-NPDase activity, up regulation of 5'-PDE activity, up regulation of 5'-PDase activity, up regulation of 5'-exonuclease activity, up regulation of 5'-nucleotide phosphodiesterase activity, up regulation of 5'-phosphodiesterase activity, up regulation of 5'NPDE activity, up regulation of alkaline phosphodiesterase activity, up regulation of exonuclease I activity, up-regulation of 5'-NPDase activity, up-regulation of 5'-PDE activity, up-regulation of 5'-PDase activity, up-regulation of 5'-exonuclease activity, up-regulation of 5'-nucleotide phosphodiesterase activity, up-regulation of 5'-phosphodiesterase activity, up-regulation of 5'NPDE activity, up-regulation of alkaline phosphodiesterase activity, up-regulation of exonuclease I activity, upregulation of 5'-NPDase activity, upregulation of 5'-PDE activity, upregulation of 5'-PDase activity, upregulation of 5'-exonuclease activity, upregulation of 5'-nucleotide phosphodiesterase activity, upregulation of 5'-phosphodiesterase activity, upregulation of 5'NPDE activity, upregulation of alkaline phosphodiesterase activity, upregulation of exonuclease I activity Relationships: is a type of positive regulation of hydrolase activity [GO:0051345]; positively regulates phosphodiesterase I activity [GO:0004528]